{
  "term_id": "GO:0030870",
  "gene": "UniProtKB:O60934",
  "gene_name": "Nibrin",
  "term_label": "Mre11 complex",
  "gene_symbol": "NBN"
}